{
  "gene_symbol": "IL32",
  "gene": "UniProtKB:P24001",
  "term_id": "UNKNOWN:0002",
  "term_label": "Unknown biological process",
  "gene_name": "Interleukin-32"
}